{
  "gene": "UniProtKB:P47869",
  "term_id": "GO:0032590",
  "gene_name": "Gamma-aminobutyric acid receptor subunit alpha-2",
  "term_label": "dendrite membrane",
  "gene_symbol": "GABRA2"
}